{
  "gene_name": "Polyisoprenoid diphosphate_phosphate phosphohydrolase PLPP6",
  "term_id": "GO:0046839",
  "gene_symbol": "PLPP6",
  "gene": "UniProtKB:Q8IY26",
  "term_label": "phospholipid dephosphorylation"
}